beta-glucosidase activity [GO:0008422] (molecular function) Definition: Catalysis of the hydrolysis of terminal, non-reducing beta-D-glucose residues with release of beta-D-glucose. References: PMID:12594539 Sources: EC:3.2.1.21 Subtypes: GO:0004338, 6-phospho-beta-glucosidase activity [GO:0008706], GO:0031217, GO:0033913, GO:0033935, beta-apiosyl-beta-glucosidase activity [GO:0033956], GO:0042973, glucan endo-1,6-beta-glucosidase activity [GO:0046557], amygdalin beta-glucosidase activity [GO:0047668], GO:0047782, prunasin beta-glucosidase activity [GO:0050224], raucaffricine beta-glucosidase activity [GO:0050247], GO:0050295, GO:0050392, strictosidine beta-glucosidase activity [GO:0050422], abscisic acid glucose ester beta-glucosidase activity [GO:0051993], cellobiose glucosidase activity [GO:0080079], 4-methylumbelliferyl-beta-D-glucopyranoside beta-glucosidase activity [GO:0080081], esculin beta-glucosidase activity [GO:0080082], GO:0080083 Relationships: is a type of glucosidase activity [GO:0015926] Also known as: beta-D-glucosidase activity, beta-glucoside glucohydrolase activity, amygdalase activity, amygdalinase, arbutinase activity, cellobiase activity, cytokine beta-glucosidase activity, elaterase activity, gentiobiase activity, gentobiase activity, limarase activity, p-nitrophenyl beta-glucosidase activity, primeverosidase activity, quercetin 3'-O-beta-D-glucopyranoside hydrolase activity, quercetin 4'-O-beta-D-glucopyranoside hydrolase activity, salicilinase activity, aryl-beta-glucosidase activity, beta-1,6-glucosidase activity, beta-D-glucoside glucohydrolase activity, emulsin